{
  "gene": "UniProtKB:O15553",
  "gene_name": "Pyrin",
  "gene_symbol": "MEFV",
  "term_id": "GO:0045087",
  "term_label": "innate immune response"
}